{
  "term_id": "GO:0005829",
  "term_label": "cytosol",
  "gene_symbol": "CALB1",
  "gene": "UniProtKB:P05937",
  "gene_name": "Calbindin"
}